{
  "term_id": "GO:0007189",
  "gene_name": "Sphingosine 1-phosphate receptor 2",
  "gene_symbol": "S1PR2",
  "gene": "UniProtKB:O95136",
  "term_label": "adenylate cyclase-activating G protein-coupled receptor signaling pathway"
}